{
  "gene": "UniProtKB:P00451",
  "term_label": "blood coagulation, intrinsic pathway",
  "term_id": "GO:0007597",
  "gene_symbol": "F8",
  "gene_name": "Coagulation factor VIII"
}